{
  "term_id": "UNKNOWN:0001",
  "gene_symbol": "CCDC59",
  "term_label": "Unknown molecular function",
  "gene_name": "Thyroid transcription factor 1-associated protein 26",
  "gene": "UniProtKB:Q9P031"
}